{
  "gene_name": "Paired box protein Pax-6",
  "gene": "UniProtKB:P26367",
  "term_label": "forebrain development",
  "term_id": "GO:0030900",
  "gene_symbol": "PAX6"
}